endothelial tip cell fate specification [GO:0097102] (biological process) Relationships: is a type of GO:0097101; BFO_0000050 sprouting angiogenesis [GO:0002040] Definition: The process involved in the specification of identity of an endothelial tip cell. Once specification has taken place, a cell will be committed to differentiate down a specific pathway if left in its normal environment. An endothelial tip cell is a specialized endothelial cell localized to the leading edge of an angiogenic sprout that senses extracellular signals and guides the directed growth of blood vessels. Also known as: angiogenic tip cell fate specification References: PMID:21521739 Sources: CL:0000704, GOC:dgh